{
  "gene": "UniProtKB:P19388",
  "term_id": "GO:0005736",
  "gene_symbol": "POLR2E",
  "gene_name": "DNA-directed RNA polymerases I, II, and III subunit RPABC1",
  "term_label": "RNA polymerase I complex"
}